negative regulation of sterol transport [GO:0032372] (biological process) Definition: Any process that stops, prevents, or reduces the frequency, rate or extent of the directed movement of sterols into, out of or within a cell, or between cells, by means of some agent such as a transporter or pore. Sources: GOC:mah Also known as: down regulation of sterol transport, down-regulation of sterol transport, downregulation of sterol transport, inhibition of sterol transport Relationships: is a type of GO:0032369; is a type of regulation of sterol transport [GO:0032371]; negatively regulates sterol transport [GO:0015918] Subtypes: negative regulation of cholesterol transport [GO:0032375], negative regulation of intracellular sterol transport [GO:0032381], GO:2000910